small nuclear ribonucleoprotein complex [GO:0030532] (cellular component) Relationships: is a type of GO:0120114; is a type of nuclear protein-containing complex [GO:0140513]; is a type of ribonucleoprotein complex [GO:1990904] Subtypes: U7 snRNP [GO:0005683], GO:0097525, 7SK snRNP [GO:0120259] Definition: A ribonucleoprotein complex that contains at least one RNA of the small nuclear RNA (snRNA) class and as well as its associated proteins. These are typically named after the snRNA(s) they contain, e.g. U1 snRNP, U4/U6 snRNP, or 7SK snRNP. Many, of these complexes become part of the spliceosome involved in splicing of nuclear mRNAs. Others are involved in regulation of transcription elongation or 3'-end processing of replication-dependent histone pre-mRNAs. Sources: GOC:krc, GOC:mah, ISBN:0879695897 Also known as: small nuclear ribonucleoprotein, snRNP